renal system vasculature morphogenesis [GO:0061438] (biological process) Definition: The process in which the renal system vasculature is generated and organized. Morphogenesis pertains to the creation of form. Relationships: is a type of anatomical structure morphogenesis [GO:0009653]; is part of renal system vasculature development [GO:0061437] References: PMID:11891195 Sources: GOC:dph, GOC:mtg_kidney_jan10